{
  "gene_symbol": "RB1",
  "term_id": "GO:0031175",
  "term_label": "neuron projection development",
  "gene": "UniProtKB:P06400",
  "gene_name": "Retinoblastoma-associated protein"
}